{
  "term_id": "UNKNOWN:0001",
  "gene": "UniProtKB:A6NJY4",
  "gene_symbol": "TMEM238L",
  "gene_name": "Transmembrane protein 238-like",
  "term_label": "Unknown molecular function"
}